{
  "term_id": "GO:0000978",
  "gene": "UniProtKB:P57082",
  "gene_symbol": "TBX4",
  "gene_name": "T-box transcription factor TBX4",
  "term_label": "RNA polymerase II cis-regulatory region sequence-specific DNA binding"
}